{
  "term_label": "structural constituent of skin epidermis",
  "gene_name": "Keratin, type II cytoskeletal 79",
  "gene_symbol": "KRT79",
  "gene": "UniProtKB:Q5XKE5",
  "term_id": "GO:0030280"
}